glucosylceramide biosynthetic process [GO:0006679] (biological process) References: PMID:35536927 Definition: The chemical reactions and pathways resulting in the formation of glucosylceramides, any compound composed of a ceramide backbone covalently linked to a glucose. The glucose can be further elongated with the sequential addition of various carbohydrate units. Relationships: is_a glucosylceramide metabolic process [GO:0006678]; is a type of GO:0006688; is a type of ceramide biosynthetic process [GO:0046513] Regulation: regulated by GO:0046317; negatively regulated by negative regulation of glucosylceramide biosynthetic process [GO:0046318]; positively regulated by positive regulation of glucosylceramide biosynthetic process [GO:0046319] Also known as: glucosylceramide anabolism, glucosylceramide biosynthesis, glucosylceramide formation, glucosylceramide synthesis